{
  "term_id": "GO:0003677",
  "gene": "UniProtKB:Q12905",
  "gene_symbol": "ILF2",
  "term_label": "DNA binding",
  "gene_name": "Interleukin enhancer-binding factor 2"
}